ovulation from ovarian follicle [GO:0001542] (biological process) Definition: The process leading to the rupture of the follicle, releasing the centrally located oocyte into the oviduct. An example of this is found in Mus musculus. Sources: GOC:mtg_sensu, https://www.ncbi.nlm.nih.gov/books/NBK279054/ Relationships: is a type of ovulation cycle process [GO:0022602]; is a type of ovulation [GO:0030728]; is part of female gonad development [GO:0008585]